{
  "term_label": "Unknown molecular function",
  "term_id": "UNKNOWN:0001",
  "gene": "UniProtKB:Q13206",
  "gene_symbol": "DDX10",
  "gene_name": "Probable ATP-dependent RNA helicase DDX10"
}